{
  "gene_name": "Zinc finger BED domain-containing protein 2",
  "term_label": "positive regulation of keratinocyte differentiation",
  "gene": "UniProtKB:Q9BTP6",
  "term_id": "GO:0045618",
  "gene_symbol": "ZBED2"
}